{
  "gene_name": "Pre-mRNA-splicing regulator WTAP",
  "gene": "UniProtKB:Q15007",
  "gene_symbol": "WTAP",
  "term_label": "regulation of alternative mRNA splicing, via spliceosome",
  "term_id": "GO:0000381"
}